{
  "gene_symbol": "PDLIM1",
  "gene_name": "PDZ and LIM domain protein 1",
  "gene": "UniProtKB:O00151",
  "term_id": "GO:0061061",
  "term_label": "muscle structure development"
}